{
  "gene_symbol": "BEST1",
  "term_id": "UNKNOWN:0001",
  "gene_name": "Bestrophin-1",
  "gene": "UniProtKB:O76090",
  "term_label": "Unknown molecular function"
}